actin filament uncapping [GO:0051695] (biological process) Sources: GOC:pf Definition: The removal of capping protein from the end of actin filaments to free the ends for addition, exchange or removal of further actin subunits. Subtypes: barbed-end actin filament uncapping [GO:0051638], pointed-end actin filament uncapping [GO:0051696] Relationships: is a type of positive regulation of actin filament depolymerization [GO:0030836] Also known as: F-actin uncapping